{
  "gene": "UniProtKB:P14866",
  "term_id": "GO:0003729",
  "gene_name": "Heterogeneous nuclear ribonucleoprotein L",
  "term_label": "mRNA binding",
  "gene_symbol": "HNRNPL"
}